{
  "gene_symbol": "MAGED4",
  "term_label": "nucleus",
  "gene": "UniProtKB:Q96JG8",
  "term_id": "GO:0005634",
  "gene_name": "Melanoma-associated antigen D4"
}